minus-end directed microtubule sliding [GO:0031534] (biological process) Definition: The movement of one microtubule along another microtubule, where the motion is directed towards the minus ends of the microtubules. Sources: GOC:mah, GOC:vw Relationships: is a type of GO:0051012